{
  "term_id": "GO:0050220",
  "term_label": "prostaglandin-E synthase activity",
  "gene_name": "Prostaglandin E synthase",
  "gene_symbol": "PTGES",
  "gene": "UniProtKB:O14684"
}